{
  "gene": "UniProtKB:P56270",
  "gene_name": "Myc-associated zinc finger protein",
  "term_label": "DNA-binding transcription factor activity, RNA polymerase II-specific",
  "term_id": "GO:0000981",
  "gene_symbol": "MAZ"
}